regulation of humoral immune response mediated by circulating immunoglobulin [GO:0002923] (biological process) Subtypes: negative regulation of humoral immune response mediated by circulating immunoglobulin [GO:0002924], positive regulation of humoral immune response mediated by circulating immunoglobulin [GO:0002925], GO:0030450 Sources: GOC:add Definition: Any process that modulates the frequency, rate, or extent of a humoral immune response mediated by circulating immunoglobulin. Relationships: is a type of regulation of immunoglobulin mediated immune response [GO:0002889]; is a type of regulation of humoral immune response [GO:0002920]; regulates humoral immune response mediated by circulating immunoglobulin [GO:0002455]